{
  "gene": "UniProtKB:Q9UH90",
  "term_id": "UNKNOWN:0001",
  "term_label": "Unknown molecular function",
  "gene_name": "F-box only protein 40",
  "gene_symbol": "FBXO40"
}